{
  "gene": "UniProtKB:Q8N3J3",
  "gene_name": "Homologous recombination OB-fold protein",
  "term_label": "Unknown molecular function",
  "term_id": "UNKNOWN:0001",
  "gene_symbol": "HROB"
}